peptidyl-histidine methylation [GO:0018021] (biological process) Sources: RESID:AA0073, RESID:AA0317 Relationships: is a type of protein methylation [GO:0006479]; is a type of peptidyl-histidine modification [GO:0018202] Subtypes: peptidyl-histidine methylation, to form tele-methylhistidine [GO:0042038] Definition: The methylation of peptidyl-L-histidine to form peptidyl-L-1'-methyl-L-histidine (otherwise known as tau-methylhistidine, tele-methylhistidine) or peptidyl-L-3'-methyl-L-histidine (otherwise known as pi-methylhistidine, pros-methylhistidine).